{
  "gene": "UniProtKB:Q9UNW9",
  "term_label": "regulation of alternative mRNA splicing, via spliceosome",
  "term_id": "GO:0000381",
  "gene_name": "RNA-binding protein Nova-2",
  "gene_symbol": "NOVA2"
}